{
  "gene_name": "U4_U6.U5 small nuclear ribonucleoprotein 27 kDa protein",
  "gene_symbol": "SNRNP27",
  "gene": "UniProtKB:Q8WVK2",
  "term_label": "Unknown cellular component",
  "term_id": "UNKNOWN:0003"
}